{
  "gene_name": "Tetraspanin-18",
  "gene_symbol": "TSPAN18",
  "term_id": "UNKNOWN:0001",
  "gene": "UniProtKB:Q96SJ8",
  "term_label": "Unknown molecular function"
}